{
  "gene": "UniProtKB:Q15831",
  "gene_name": "Serine_threonine-protein kinase STK11",
  "gene_symbol": "STK11",
  "term_id": "GO:0006974",
  "term_label": "DNA damage response"
}